outflow tract morphogenesis [GO:0003151] (biological process) Sources: GOC:mtg_heart, UBERON:0004145 Definition: The process in which the anatomical structures of the outflow tract are generated and organized. The outflow tract is the portion of the heart through which blood flows into the arteries. Relationships: is a type of anatomical structure morphogenesis [GO:0009653]; is part of heart morphogenesis [GO:0003007]